{
  "term_label": "JUN kinase phosphatase activity",
  "gene_name": "Dual specificity protein phosphatase 19",
  "term_id": "GO:0008579",
  "gene": "UniProtKB:Q8WTR2",
  "gene_symbol": "DUSP19"
}